{
  "gene_symbol": "HMGN3",
  "gene_name": "High mobility group nucleosome-binding domain-containing protein 3",
  "term_label": "nucleus",
  "term_id": "GO:0005634",
  "gene": "UniProtKB:Q15651"
}